{
  "gene_symbol": "AIF1",
  "term_label": "ruffle membrane",
  "term_id": "GO:0032587",
  "gene_name": "Allograft inflammatory factor 1",
  "gene": "UniProtKB:P55008"
}